{
  "term_id": "GO:0045892",
  "term_label": "negative regulation of DNA-templated transcription",
  "gene_symbol": "CIPC",
  "gene_name": "CLOCK-interacting pacemaker",
  "gene": "UniProtKB:Q9C0C6"
}